translation elongation factor binding [GO:0061770] (molecular function) Sources: GOC:dph Relationships: is a type of protein binding [GO:0005515] Definition: Binding to a translation elongation factor, any polypeptide factor involved in the peptide elongation in ribosome-mediated translation.